mesenchymal cell differentiation involved in lung development [GO:0060915] (biological process) Sources: GOC:dph Relationships: is a type of mesenchymal cell differentiation [GO:0048762]; is part of GO:0030324 Definition: The process in which a relatively unspecialized cell acquires specialized features of a mesenchymal cell of the lung. A mesenchymal cell is a loosely associated cell that is part of the connective tissue in an organism. Mesenchymal cells give rise to more mature connective tissue cell types.